{
  "term_id": "GO:0005254",
  "gene_name": "Gamma-aminobutyric acid receptor subunit gamma-2",
  "term_label": "chloride channel activity",
  "gene_symbol": "GABRG2",
  "gene": "UniProtKB:P18507"
}